{
  "gene": "UniProtKB:P61769",
  "term_id": "GO:0050778",
  "gene_name": "Beta-2-microglobulin",
  "term_label": "positive regulation of immune response",
  "gene_symbol": "B2M"
}